{
  "gene_symbol": "ACVR1",
  "term_label": "transforming growth factor beta receptor signaling pathway",
  "term_id": "GO:0007179",
  "gene_name": "Activin receptor type-1",
  "gene": "UniProtKB:Q04771"
}